{
  "gene": "UniProtKB:Q8TB24",
  "term_label": "cytosol",
  "gene_symbol": "RIN3",
  "gene_name": "Ras and Rab interactor 3",
  "term_id": "GO:0005829"
}